positive regulation of protein localization to basolateral plasma membrane [GO:1904510] (biological process) Also known as: positive regulation of protein localisation in basolateral plasma membrane, positive regulation of protein localisation to basolateral plasma membrane, positive regulation of protein localization in basolateral plasma membrane, up regulation of protein localisation in basolateral plasma membrane, up regulation of protein localisation to basolateral plasma membrane, up regulation of protein localization in basolateral plasma membrane, up regulation of protein localization to basolateral plasma membrane, up-regulation of protein localisation in basolateral plasma membrane, up-regulation of protein localisation to basolateral plasma membrane, up-regulation of protein localization in basolateral plasma membrane, up-regulation of protein localization to basolateral plasma membrane, upregulation of protein localisation in basolateral plasma membrane, upregulation of protein localisation to basolateral plasma membrane, upregulation of protein localization in basolateral plasma membrane, upregulation of protein localization to basolateral plasma membrane, activation of protein localisation in basolateral plasma membrane, activation of protein localisation to basolateral plasma membrane, activation of protein localization in basolateral plasma membrane, activation of protein localization to basolateral plasma membrane References: PMID:26115433 Sources: GOC:TermGenie, GOC:kmv, GO_REF:0000058 Relationships: is a type of positive regulation of protein localization to cell periphery [GO:1904377]; is a type of regulation of protein localization to basolateral plasma membrane [GO:1904508]; is a type of positive regulation of protein localization to membrane [GO:1905477]; positively regulates protein localization to basolateral plasma membrane [GO:1903361] Definition: Any process that activates or increases the frequency, rate or extent of protein localization to basolateral plasma membrane.